D-gluconate metabolic process [GO:0019521] (biological process) Subtypes: D-gluconate biosynthetic process [GO:0046178] Sources: ISBN:0198506732 Also known as: D-gluconate metabolism Definition: The chemical reactions and pathways involving D-gluconate, the anion of D-gluconic acid, the aldonic acid derived from glucose. Relationships: is_a carbohydrate metabolic process [GO:0005975]; is a type of monocarboxylic acid metabolic process [GO:0032787]